Lugaro cell differentiation [GO:0021708] (biological process) Relationships: is a type of GO:0021533; is a type of GO:0021953; is_a GO:0097154; is part of cerebellar cortex formation [GO:0021697] Definition: The process in which neuroblasts acquire specialized structural and/or functional features that characterize the mature Lugaro cell. Differentiation includes the processes involved in commitment of a neuroblast to a Lugaro cell fate. A Lugaro cell is an inhibitory GABAergic interneuron found in the cerebellar cortex. References: PMID:15157725 Sources: GOC:cls, GOC:dgh, GOC:dph, GOC:jid, GO_REF:0000021